{
  "term_id": "GO:0051017",
  "gene_name": "Plastin-1",
  "term_label": "actin filament bundle assembly",
  "gene_symbol": "PLS1",
  "gene": "UniProtKB:Q14651"
}